{
  "gene_name": "Zinc finger protein 174",
  "term_id": "UNKNOWN:0003",
  "gene_symbol": "ZNF174",
  "term_label": "Unknown cellular component",
  "gene": "UniProtKB:Q15697"
}